{
  "term_label": "Unknown biological process",
  "gene_name": "Complement component C8 gamma chain",
  "gene": "UniProtKB:P07360",
  "gene_symbol": "C8G",
  "term_id": "UNKNOWN:0002"
}